female pregnancy [GO:0007565] (biological process) Definition: The set of physiological processes that allow an embryo or foetus to develop within the body of a female animal. It covers the time from fertilization of a female ovum by a male spermatozoon until birth. Sources: ISBN:0192800825 Relationships: is a type of multi-organism reproductive process [GO:0044703]; is a type of multi-multicellular organism process [GO:0044706] Also known as: gestation, carrying of young